{
  "gene": "UniProtKB:Q5FYB1",
  "gene_symbol": "ARSI",
  "term_id": "GO:0008484",
  "term_label": "sulfuric ester hydrolase activity",
  "gene_name": "Arylsulfatase I"
}